{
  "gene_name": "Amiloride-sensitive sodium channel subunit gamma",
  "term_id": "GO:0035725",
  "gene_symbol": "SCNN1G",
  "gene": "UniProtKB:P51170",
  "term_label": "sodium ion transmembrane transport"
}